{
  "term_label": "Ino80 complex",
  "gene_name": "INO80 complex subunit E",
  "gene": "UniProtKB:Q8NBZ0",
  "term_id": "GO:0031011",
  "gene_symbol": "INO80E"
}